{
  "term_id": "GO:0002769",
  "gene_symbol": "CLEC12B",
  "gene_name": "C-type lectin domain family 12 member B",
  "gene": "UniProtKB:Q2HXU8",
  "term_label": "natural killer cell inhibitory signaling pathway"
}